{
  "gene": "UniProtKB:Q9UKY1",
  "gene_name": "Zinc fingers and homeoboxes protein 1",
  "term_id": "GO:0000981",
  "term_label": "DNA-binding transcription factor activity, RNA polymerase II-specific",
  "gene_symbol": "ZHX1"
}